{
  "gene_symbol": "STXBP4",
  "term_id": "GO:0008286",
  "term_label": "insulin receptor signaling pathway",
  "gene_name": "Syntaxin-binding protein 4",
  "gene": "UniProtKB:Q6ZWJ1"
}